{
  "term_label": "Unknown biological process",
  "gene": "UniProtKB:Q5BKY6",
  "gene_symbol": "Q5BKY6",
  "term_id": "UNKNOWN:0002",
  "gene_name": "Putative uncharacterized protein DKFZp434K191"
}